positive regulation of dauer larval development [GO:0061066] (biological process) Sources: GOC:dph, GOC:kmv Definition: Any process that increases the rate, frequency, or extent of dauer larval development, the process whose specific outcome is the progression of the dauer larva over time, through the facultative diapause of the dauer (enduring) larval stage, with specialized traits adapted for dispersal and long-term survival, with elevated stress resistance and without feeding. Relationships: is a type of positive regulation of nematode larval development [GO:0061063]; is a type of regulation of dauer larval development [GO:0061065]; positively regulates dauer larval development [GO:0040024]